endoplasmic reticulum tubular network [GO:0071782] (cellular component) Definition: A subcompartment of the endoplasmic reticulum consisting of tubules having membranes with high curvature in cross-section. References: PMID:16469703, PMID:20434336 Sources: GOC:vw Relationships: is a type of endoplasmic reticulum subcompartment [GO:0098827] Also known as: ER tubular network Subtypes: cortical endoplasmic reticulum [GO:0032541]